antigen processing and presentation of endogenous peptide antigen via MHC class Ib [GO:0002476] (biological process) References: PMID:15928678 Sources: GOC:add Definition: The process in which an antigen-presenting cell expresses a peptide antigen of endogenous origin on its cell surface in association with an MHC class Ib protein complex. The peptide is typically a fragment of a larger endogenous protein which has been degraded within the cell. Class Ib here refers to non-classical class I molecules, such as those of the HLA-E gene family. Also known as: endogenous peptide antigen processing and presentation via MHC class Ib Relationships: is a type of antigen processing and presentation of peptide antigen via MHC class Ib [GO:0002428]; is a type of antigen processing and presentation of endogenous peptide antigen [GO:0002483] Subtypes: antigen processing and presentation of endogenous peptide antigen via MHC class Ib via ER pathway [GO:0002488]